tRNA pseudouridylation guide activity [GO:0030560] (molecular function) Note: Note that this term describes the activity of a nucleic acid, usually RNA, gene product that interacts with other RNA molecules via base pairing; it should not be used to annotate proteins. Definition: Specifies the site of pseudouridylation in a tRNA molecule by base pairing with a short sequence around the target residue. Relationships: is a type of GO:0030557; is a type of RNA pseudouridylation guide activity [GO:0030558] References: PMID:12457565 Sources: GOC:mah